calcium export from the mitochondrion [GO:0099093] (biological process) Relationships: is a type of mitochondrial calcium ion transmembrane transport [GO:0006851]; is a type of release of sequestered calcium ion into cytosol [GO:0051209] Also known as: mitochondrial calcium ion export, calcium ion transmembrane export from mitochondrion, mitochondrial calcium release Subtypes: calcium export from the mitochondrion involved in positive regulation of presynaptic cytosolic calcium concentration [GO:1905741] Definition: A process in which a calcium ion (Ca2+) is transported out of the mitochondrial matrix, and into the cytosol. Sources: GOC:dos, GOC:vw